benzoate-CoA ligase activity [GO:0018858] (molecular function) Sources: EC:6.2.1.25, RHEA:10132 Also known as: benzoate-coenzyme A ligase activity, benzoate:CoA ligase (AMP-forming), benzoyl CoA synthetase (AMP forming), benzoyl-coenzyme A synthetase activity Relationships: is a type of GO:0016405; is a type of acid-thiol ligase activity [GO:0016878] Definition: Catalysis of the reaction: ATP + benzoate + CoA = AMP + benzoyl-CoA + diphosphate.